{
  "gene_name": "Protein Wnt-10a",
  "gene_symbol": "WNT10A",
  "gene": "UniProtKB:Q9GZT5",
  "term_id": "GO:0030182",
  "term_label": "neuron differentiation"
}